7,8-didemethyl-8-hydroxy-5-deazariboflavin catabolic process [GO:1901851] (biological process) Relationships: is a type of GO:0009056 Definition: The chemical reactions and pathways resulting in the breakdown of 7,8-didemethyl-8-hydroxy-5-deazariboflavin. Also known as: 7,8-didemethyl-8-hydroxy-5-deazariboflavin breakdown, 7,8-didemethyl-8-hydroxy-5-deazariboflavin catabolism, 7,8-didemethyl-8-hydroxy-5-deazariboflavin degradation, coenzyme F0 breakdown, coenzyme F0 catabolic process, coenzyme F0 catabolism, coenzyme F0 degradation References: PMID:14593448 Sources: GOC:TermGenie, GOC:yaf, UniPathway:UPA00072